{
  "term_label": "centriole",
  "gene_name": "Centriolar coiled-coil protein of 110 kDa",
  "gene": "UniProtKB:O43303",
  "term_id": "GO:0005814",
  "gene_symbol": "CCP110"
}